{
  "gene": "UniProtKB:Q5VX52",
  "term_label": "Unknown biological process",
  "gene_symbol": "SPATA1",
  "term_id": "UNKNOWN:0002",
  "gene_name": "Spermatogenesis-associated protein 1"
}